positive regulation of ent-pimara-8(14),15-diene biosynthetic process [GO:1901544] (biological process) Sources: GOC:TermGenie, GOC:di Relationships: is_a positive regulation of lipid biosynthetic process [GO:0046889]; is_a GO:1901542; positively regulates GO:1901541 Also known as: positive regulation of ent-pimara-8(14),15-diene anabolism, positive regulation of ent-pimara-8(14),15-diene biosynthesis, positive regulation of ent-pimara-8(14),15-diene formation, positive regulation of ent-pimara-8(14),15-diene synthesis, up regulation of ent-pimara-8(14),15-diene anabolism, up regulation of ent-pimara-8(14),15-diene biosynthesis, up regulation of ent-pimara-8(14),15-diene biosynthetic process, up regulation of ent-pimara-8(14),15-diene formation, up regulation of ent-pimara-8(14),15-diene synthesis, up-regulation of ent-pimara-8(14),15-diene anabolism, up-regulation of ent-pimara-8(14),15-diene biosynthesis, up-regulation of ent-pimara-8(14),15-diene biosynthetic process, up-regulation of ent-pimara-8(14),15-diene formation, up-regulation of ent-pimara-8(14),15-diene synthesis, upregulation of ent-pimara-8(14),15-diene anabolism, upregulation of ent-pimara-8(14),15-diene biosynthesis, upregulation of ent-pimara-8(14),15-diene biosynthetic process, upregulation of ent-pimara-8(14),15-diene formation, upregulation of ent-pimara-8(14),15-diene synthesis, activation of ent-pimara-8(14),15-diene anabolism, activation of ent-pimara-8(14),15-diene biosynthesis, activation of ent-pimara-8(14),15-diene biosynthetic process, activation of ent-pimara-8(14),15-diene formation, activation of ent-pimara-8(14),15-diene synthesis Definition: Any process that activates or increases the frequency, rate or extent of ent-pimara-8(14),15-diene biosynthetic process.